{
  "gene_symbol": "DKKL1",
  "gene_name": "Dickkopf-like protein 1",
  "gene": "UniProtKB:Q9UK85",
  "term_id": "GO:0090090",
  "term_label": "negative regulation of canonical Wnt signaling pathway"
}